{
  "gene_name": "Threonylcarbamoyladenosine tRNA methylthiotransferase",
  "gene_symbol": "CDKAL1",
  "gene": "UniProtKB:Q5VV42",
  "term_id": "GO:0005783",
  "term_label": "endoplasmic reticulum"
}